histamine production involved in inflammatory response [GO:0002349] (biological process) Relationships: is a type of production of molecular mediator involved in inflammatory response [GO:0002532] Definition: The synthesis or release of histamine following a stimulus as part of an inflammatory response, resulting in an increase in its intracellular or extracellular levels. References: PMID:16730260 Sources: GOC:add, ISBN:0781735149 Also known as: histamine production involved in acute inflammatory response